{
  "gene_symbol": "C1QB",
  "gene_name": "Complement C1q subcomponent subunit B",
  "gene": "UniProtKB:P02746",
  "term_label": "Unknown biological process",
  "term_id": "UNKNOWN:0002"
}